cell migration involved in heart jogging [GO:0003305] (biological process) Sources: GOC:mtg_heart Relationships: is a type of cell migration involved in heart development [GO:0060973]; is part of GO:0003146 Definition: The orderly movement of a cell of the myocardium from one site to another that will contribute to heart jogging.